{
  "term_id": "GO:0006283",
  "term_label": "transcription-coupled nucleotide-excision repair",
  "gene": "UniProtKB:Q13216",
  "gene_symbol": "ERCC8",
  "gene_name": "DNA excision repair protein ERCC-8"
}